regulation of myofibroblast contraction [GO:1904328] (biological process) Definition: Any process that modulates the frequency, rate or extent of myofibroblast contraction. Subtypes: GO:1904329, positive regulation of myofibroblast contraction [GO:1904330] Also known as: regulation of MF contraction, regulation of MFB contraction Relationships: is a type of regulation of actin filament-based movement [GO:1903115]; regulates GO:1990764 References: PMID:19239477 Sources: GOC:TermGenie, GO_REF:0000058